{
  "gene": "UniProtKB:Q9H4Z3",
  "gene_name": "mRNA (2'-O-methyladenosine-N(6)-)-methyltransferase",
  "term_label": "nucleus",
  "term_id": "GO:0005634",
  "gene_symbol": "PCIF1"
}